type IV pilus assembly [GO:0043683] (biological process) Relationships: is a type of pilus assembly [GO:0009297] Also known as: type IV fimbria assembly, type IV fimbria biogenesis, type IV fimbriae assembly, type IV fimbriae biogenesis, type IV fimbrial assembly, type IV fimbrial biogenesis, type IV fimbrium assembly, type IV fimbrium biogenesis, type IV pilus biogenesis Definition: The assembly from its constituent parts of a type IV pilus. Regulation: regulated by regulation of type IV pilus biogenesis [GO:1903656]; negatively regulated by negative regulation of type IV pilus biogenesis [GO:1903657]; positively regulated by positive regulation of type IV pilus biogenesis [GO:1903658] References: PMID:31784891 Sources: GOC:jl, GOC:ml